{
  "gene": "UniProtKB:Q13285",
  "term_label": "regulation of transcription by RNA polymerase II",
  "gene_name": "Steroidogenic factor 1",
  "term_id": "GO:0006357",
  "gene_symbol": "NR5A1"
}